cysteamine dioxygenase activity [GO:0047800] (molecular function) Definition: Catalysis of the reaction: cysteamine + O2 = H+ + hypotaurine. Sources: EC:1.13.11.19, RHEA:14409 Relationships: is a type of oxidoreductase activity, acting on single donors with incorporation of molecular oxygen, incorporation of two atoms of oxygen [GO:0016702] Also known as: 2-aminoethanethiol:oxygen oxidoreductase activity, cysteamine oxygenase activity, cysteamine:oxygen oxidoreductase activity, persulfurase activity